{
  "gene_name": "Inactive pancreatic lipase-related protein 1",
  "gene_symbol": "PNLIPRP1",
  "gene": "UniProtKB:P54315",
  "term_id": "GO:0019433",
  "term_label": "triglyceride catabolic process"
}